embryonic caudal fin morphogenesis [GO:0035124] (biological process) Sources: GOC:dgh Relationships: is_a embryonic medial fin morphogenesis [GO:0035122]; is a type of caudal fin morphogenesis [GO:0035143] Definition: The process, occurring in the embryo, by which the anatomical structures of the caudal fin are generated and organized. The caudal fin is an unpaired medial fin mounted at the caudal end of the fish and is the main fin used for propulsion.